{
  "term_label": "Unknown molecular function",
  "gene_name": "Keratin-associated protein 4-2",
  "term_id": "UNKNOWN:0001",
  "gene": "UniProtKB:Q9BYR5",
  "gene_symbol": "KRTAP4-2"
}